{
  "gene": "UniProtKB:Q9BPX5",
  "term_id": "GO:0034314",
  "gene_name": "Actin-related protein 2_3 complex subunit 5-like protein",
  "gene_symbol": "ARPC5L",
  "term_label": "Arp2/3 complex-mediated actin nucleation"
}